interleukin-22-mediated signaling pathway [GO:0140865] (biological process) Definition: The series of molecular signals initiated by interleukin-22 binding to its receptor on the surface of a target cell, and ending with the regulation of a downstream cellular process, e.g. transcription. References: PMID:34755534 Also known as: IL-22-mediated signaling pathway, interleukin-22-mediated signalling pathway Relationships: is a type of cytokine-mediated signaling pathway [GO:0019221]